{
  "gene_name": "Prothymosin alpha",
  "term_id": "GO:0005634",
  "term_label": "nucleus",
  "gene_symbol": "PTMA",
  "gene": "UniProtKB:P06454"
}